{
  "term_label": "cytoplasm",
  "gene_name": "Rho GTPase-activating protein 29",
  "gene": "UniProtKB:Q52LW3",
  "term_id": "GO:0005737",
  "gene_symbol": "ARHGAP29"
}